{
  "term_label": "axoneme",
  "term_id": "GO:0005930",
  "gene": "UniProtKB:Q8IWN7",
  "gene_name": "Retinitis pigmentosa 1-like 1 protein",
  "gene_symbol": "RP1L1"
}